short-day photoperiodism [GO:0048572] (biological process) Sources: GOC:jid, GOC:pj, ISBN:0582015952, ISBN:0697037754, ISBN:0709408862 Definition: Any process that results in a change in state or activity of an organism (in terms of movement, secretion, enzyme production, gene expression, etc.) as a result of detection of, or exposure to, a day length that falls short of a particular duration known as the 'critical day length'. The critical day length varies between species. Although the term short-day is used, most species actually respond to the duration of the night, so that the response will occur when a period of darkness exceeds the number of hours defined by 24 hours minus the critical day length. Subtypes: short-day photoperiodism, flowering [GO:0048575] Also known as: long-night photoperiodism, response to long-night, response to short-day, response to short-day photoperiod Relationships: is a type of GO:0009648